{
  "gene_name": "Cyclic nucleotide-gated cation channel alpha-3",
  "gene_symbol": "CNGA3",
  "term_id": "GO:0098655",
  "term_label": "monoatomic cation transmembrane transport",
  "gene": "UniProtKB:Q16281"
}